{
  "term_id": "GO:0034274",
  "term_label": "Atg12-Atg5-Atg16 complex",
  "gene": "UniProtKB:O94817",
  "gene_symbol": "ATG12",
  "gene_name": "Ubiquitin-like protein ATG12"
}